{
  "gene_name": "Myogenic factor 5",
  "gene_symbol": "MYF5",
  "term_label": "skeletal muscle cell differentiation",
  "gene": "UniProtKB:P13349",
  "term_id": "GO:0035914"
}